cellular response to dithiothreitol [GO:0072721] (biological process) Sources: GOC:mah Relationships: is a type of response to dithiothreitol [GO:0072720]; is a type of cellular response to oxygen-containing compound [GO:1901701] Also known as: cellular response to 1,4-dithiothreitol, cellular response to DTT Definition: Any process that results in a change in state or activity of a cell (in terms of movement, secretion, enzyme production, gene expression, etc.) as a result of a dithiothreitol stimulus.